{
  "gene_name": "UDP-glucuronosyltransferase 1A10",
  "term_id": "GO:0016125",
  "term_label": "sterol metabolic process",
  "gene_symbol": "UGT1A10",
  "gene": "UniProtKB:Q9HAW8"
}